{
  "gene_symbol": "THAP6",
  "gene_name": "THAP domain-containing protein 6",
  "term_label": "Unknown biological process",
  "gene": "UniProtKB:Q8TBB0",
  "term_id": "UNKNOWN:0002"
}